G-rich single-stranded DNA binding [GO:1990955] (molecular function) References: PMID:8493094 Sources: GOC:hjd Definition: Binding to G-rich, single-stranded DNA. Relationships: is a type of single-stranded DNA binding [GO:0003697]